cellular response to GW 7647 [GO:0072760] (BP) Relationships: is a type of response to GW 7647 [GO:1901593] Definition: Any process that results in a change in state or activity of a cell (in terms of movement, secretion, enzyme production, gene expression, etc.) as a result of a GW 7647 stimulus. Sources: GOC:mah